cellular response to sterol depletion [GO:0071501] (biological process) Relationships: is a type of response to sterol depletion [GO:0006991]; is a type of cellular response to stress [GO:0033554] Sources: GOC:mah Subtypes: SREBP signaling pathway [GO:0032933] Definition: Any process that results in a change in state or activity of a cell (in terms of movement, secretion, enzyme production, gene expression, etc.) as a result of a stimulus indicating deprivation of sterols. Sterols are a group of steroids characterized by the presence of one or more hydroxyl groups and a hydrocarbon side-chain in the molecule. Also known as: cellular sterol depletion response